{
  "gene_name": "Copine-2",
  "term_id": "GO:0005886",
  "term_label": "plasma membrane",
  "gene_symbol": "CPNE2",
  "gene": "UniProtKB:Q96FN4"
}